{
  "gene": "UniProtKB:Q96BZ9",
  "term_id": "GO:0006888",
  "term_label": "endoplasmic reticulum to Golgi vesicle-mediated transport",
  "gene_symbol": "TBC1D20",
  "gene_name": "TBC1 domain family member 20"
}